{
  "gene": "UniProtKB:P49959",
  "term_label": "double-strand break repair via nonhomologous end joining",
  "gene_name": "Double-strand break repair protein MRE11",
  "gene_symbol": "MRE11",
  "term_id": "GO:0006303"
}